{
  "gene": "UniProtKB:Q9UHJ9",
  "gene_symbol": "PGAP2",
  "term_label": "GPI anchor biosynthetic process",
  "term_id": "GO:0006506",
  "gene_name": "Post-GPI attachment to proteins factor 2"
}